regulation of fever generation by regulation of prostaglandin secretion [GO:0071810] (biological process) Sources: GOC:BHF, GOC:dph, GOC:mah Relationships: is a type of GO:0031620; is a type of regulation of prostaglandin secretion [GO:0032306]; regulates regulation of fever generation by prostaglandin secretion [GO:0100009] Definition: Any process that modulates the rate or extent of fever generation via regulation of the frequency, rate or extent of the regulated release of a prostaglandin from a cell.